lagging strand initiation [GO:0090629] (biological process) Relationships: is a type of DNA metabolic process [GO:0006259]; BFO_0000050 lagging strand elongation [GO:0006273] Definition: The process in which the synthesis of DNA from a template strand in a net 3' to 5' direction is started. Sources: GOC:mah, GOC:tb